{
  "gene_name": "WASH complex subunit 1",
  "term_label": "WASH complex",
  "gene": "UniProtKB:A8K0Z3",
  "gene_symbol": "WASHC1",
  "term_id": "GO:0071203"
}